{
  "gene_symbol": "SELENBP1",
  "gene_name": "Methanethiol oxidase",
  "gene": "UniProtKB:Q13228",
  "term_label": "Unknown molecular function",
  "term_id": "UNKNOWN:0001"
}